{
  "gene": "UniProtKB:Q5VWM4",
  "gene_name": "PRAME family member 8",
  "gene_symbol": "PRAMEF8",
  "term_id": "GO:0005737",
  "term_label": "cytoplasm"
}